{
  "term_id": "UNKNOWN:0002",
  "gene_symbol": "UCK2",
  "gene_name": "Uridine-cytidine kinase 2",
  "gene": "UniProtKB:Q9BZX2",
  "term_label": "Unknown biological process"
}